{
  "gene_name": "General transcription factor IIH subunit 3",
  "gene_symbol": "GTF2H3",
  "term_label": "nucleotide-excision repair",
  "term_id": "GO:0006289",
  "gene": "UniProtKB:Q13889"
}